{
  "gene_name": "Plexin-A1",
  "gene_symbol": "PLXNA1",
  "gene": "UniProtKB:Q9UIW2",
  "term_id": "GO:0002116",
  "term_label": "semaphorin receptor complex"
}